cellular response to diacyl bacterial lipopeptide [GO:0071726] (biological process) Also known as: cellular response to diacylated bacterial lipoprotein Note: Note that bacterial lipopeptides are derived from bacterial lipoproteins, but the two terms are sometimes used interchangeably in the literature. Relationships: is a type of GO:0071221; is a type of response to diacyl bacterial lipopeptide [GO:0071724] Definition: Any process that results in a change in state or activity of a cell (in terms of movement, secretion, enzyme production, gene expression, etc.) as a result of a diacylated bacterial lipopeptide stimulus. References: PMID:12077222, PMID:12524386, PMID:2757794 Sources: GOC:add